vagus nerve maturation [GO:0021643] (biological process) Also known as: CN X maturation Definition: A developmental process, independent of morphogenetic (shape) change, that is required for the vagus nerve to attain its fully functional state. This nerve is primarily sensory but also has visceromotor components. It originates in the brain stem and controls many autonomic functions of the heart, lungs, stomach, pharynx, larynx, trachea, esophagus and other gastrointestinal tract components. It controls some motor functions such as speech. The sensory branches mediate sensation from the pharynx, larynx, thorax and abdomen; it also innervates taste buds in the epiglottis. Sources: GOC:cls, GOC:dgh, GOC:dph, GOC:jid, GO_REF:0000021 Relationships: is a type of cranial nerve maturation [GO:0021605]; is part of vagus nerve development [GO:0021564]